{
  "gene_name": "Neutrophil defensin 1",
  "gene_symbol": "DEFA1B",
  "term_label": "antibacterial humoral response",
  "gene": "UniProtKB:P59665",
  "term_id": "GO:0019731"
}